ribosomal protein S6 kinase activity [GO:0004711] (molecular function) References: PMID:9822608 Sources: GOC:mah Relationships: is a type of protein serine/threonine kinase activity [GO:0004674] Definition: Catalysis of the reaction: ribosomal protein S6 + ATP = ribosomal protein S6 phosphate + ATP.